{
  "gene": "UniProtKB:Q8N3Z0",
  "term_id": "UNKNOWN:0001",
  "gene_name": "Inactive serine protease 35",
  "term_label": "Unknown molecular function",
  "gene_symbol": "PRSS35"
}